mitotic spindle kinetochore microtubule [GO:1990941] (cellular component) Relationships: is a type of kinetochore microtubule [GO:0005828]; is a type of mitotic spindle microtubule [GO:1990498] References: PMID:18256284 Definition: Any of the mitotic spindle microtubules that attach to the kinetochores of chromosomes by their plus ends, and maneuver the chromosomes during mitotic chromosome segregation.